{
  "gene_symbol": "GNA11",
  "gene_name": "Guanine nucleotide-binding protein subunit alpha-11",
  "term_label": "phospholipase C-activating dopamine receptor signaling pathway",
  "term_id": "GO:0060158",
  "gene": "UniProtKB:P29992"
}